{
  "gene": "UniProtKB:O00631",
  "term_id": "UNKNOWN:0002",
  "gene_symbol": "SLN",
  "gene_name": "Sarcolipin",
  "term_label": "Unknown biological process"
}